nitrilase activity [GO:0000257] (molecular function) Relationships: is a type of hydrolase activity, acting on carbon-nitrogen (but not peptide) bonds, in nitriles [GO:0016815] Also known as: acetonitrilase activity, benzonitrilase activity, nitrile aminohydrolase activity Subtypes: bromoxynil nitrilase activity [GO:0018761], aliphatic nitrilase activity [GO:0018762], GO:0047426, cyanoalanine nitrilase activity [GO:0047427], GO:0047428, GO:0080061 Definition: Catalysis of the reaction: a nitrile + H2O = a carboxylate + NH3. Acts on a wide range of aromatic nitriles including (indole-3-yl)-acetonitrile and some aliphatic nitriles, and on the corresponding acid amides. Sources: EC:3.5.5.1, GOC:kd